positive regulation of nematode larval development [GO:0061063] (biological process) Sources: GOC:dph, GOC:kmv Subtypes: positive regulation of dauer larval development [GO:0061066], positive regulation of nematode larval development, heterochronic [GO:0090445] Relationships: is a type of positive regulation of post-embryonic development [GO:0048582]; is a type of GO:0061062; positively regulates nematode larval development [GO:0002119] Definition: Any process that increases the rate, frequency, or extent of nematode larval development, the process whose specific outcome is the progression of the nematode larva over time, from its formation to the mature structure. Nematode larval development begins with the newly hatched first-stage larva (L1) and ends with the end of the last larval stage (for example the fourth larval stage (L4) in C. elegans). Each stage of nematode larval development is characterized by proliferation of specific cell lineages and an increase in body size without alteration of the basic body plan. Nematode larval stages are separated by molts in which each stage-specific exoskeleton, or cuticle, is shed and replaced anew.